{
  "gene": "UniProtKB:Q8WWZ3",
  "gene_name": "Ectodysplasin-A receptor-associated adapter protein",
  "term_id": "UNKNOWN:0001",
  "gene_symbol": "EDARADD",
  "term_label": "Unknown molecular function"
}